{
  "gene": "UniProtKB:Q14258",
  "gene_name": "E3 ubiquitin_ISG15 ligase TRIM25",
  "gene_symbol": "TRIM25",
  "term_label": "Unknown cellular component",
  "term_id": "UNKNOWN:0003"
}